lung lobe formation [GO:0060464] (BP) Relationships: is a type of anatomical structure formation involved in morphogenesis [GO:0048646]; is part of lung lobe morphogenesis [GO:0060463] Definition: The developmental process pertaining to the initial formation of a lung lobe from unspecified parts. This process begins with the specific processes that contribute to the appearance of the lobe and ends when the structural rudiment is recognizable. A lung lobe is a projection that extends from the lung. Sources: GOC:dph